{
  "term_label": "DNA-binding transcription factor activity, RNA polymerase II-specific",
  "gene": "UniProtKB:P61371",
  "gene_symbol": "ISL1",
  "term_id": "GO:0000981",
  "gene_name": "Insulin gene enhancer protein ISL-1"
}